NEDD8 conjugating enzyme activity [GO:0061654] (molecular function) Definition: Isoenergetic transfer of NEDD8 from one protein to another via the reaction X-NEDD8 + Y = Y-NEDD8 + X, where both the X-NEDD8 and Y-NEDD8 linkages are thioester bonds between the C-terminal amino acid of NEDD8 and a sulfhydryl side group of a cysteine residue. Also known as: E2 Relationships: is a type of GO:0019788; is a type of ubiquitin-like protein conjugating enzyme activity [GO:0061650] Sources: GOC:dph